DNA-templated DNA replication maintenance of fidelity [GO:0045005] (biological process) Subtypes: replication fork processing [GO:0031297], replication fork arrest [GO:0043111], DNA replication proofreading [GO:0045004], GO:1902298 Sources: GOC:mah, GOC:vw Definition: A DNA metabolic process that prevents or corrects errors to ensure that DNA is replicated accurately. Errors can be corrected either by intrinsic DNA polymerase proofreading activity or via mismatch repair. Relationships: is a type of DNA metabolic process [GO:0006259]; is part of DNA-templated DNA replication [GO:0006261] Also known as: DNA-dependent DNA replication maintenance of fidelity, maintenance of fidelity involved in DNA-dependent DNA replication, maintenance of fidelity during DNA-dependent DNA replication